metalloendopeptidase inhibitor activity [GO:0008191] (molecular function) Sources: GOC:ai Also known as: metalloprotease inhibitor, metalloproteinase inhibitor Definition: Binds to and stops, prevents or reduces the activity of metalloendopeptidases, enzymes that catalyze the hydrolysis of nonterminal peptide bonds in a polypeptide chain and contain a chelated metal ion at their active sites which is essential to their catalytic activity. Relationships: is a type of endopeptidase inhibitor activity [GO:0004866]; negatively regulates metalloendopeptidase activity [GO:0004222]